ABC-type alkanesulfonate transporter transporter activity [GO:0042959] (molecular function) Relationships: is a type of ABC-type transporter activity [GO:0140359]; is_a sulfur compound transmembrane transporter activity [GO:1901682]; is part of alkanesulfonate transmembrane transport [GO:0042918] Definition: Enables the transfer of an alkanesulfonate from one side of a membrane to the other according to the reaction: ATP + H2O + alkanesulfonate(out) = ADP + phosphate + alkanesulfonate(in). Subtypes: GO:0015411 Also known as: alkanesulfonate transmembrane transporter activity, alkanesulphonate transporter activity, alkanesulfonate transporter activity References: PMID:10506196